scutellarein 7-methyl ether 6-O-methyltransferase activity [GO:0102623] (molecular function) Definition: Catalysis of the reaction: S-adenosyl-L-methionine + scutellarein 7-methyl ether = cirsimaritin + H+ + S-adenosyl-L-homocysteine. Sources: RHEA:73243 Relationships: is a type of GO:0008168